{
  "term_label": "camera-type eye development",
  "term_id": "GO:0043010",
  "gene_symbol": "NEUROD4",
  "gene": "UniProtKB:Q9HD90",
  "gene_name": "Neurogenic differentiation factor 4"
}